{
  "gene": "UniProtKB:P43361",
  "gene_name": "Melanoma-associated antigen 8",
  "term_id": "GO:0000122",
  "gene_symbol": "MAGEA8",
  "term_label": "negative regulation of transcription by RNA polymerase II"
}